{
  "term_label": "lagging strand elongation",
  "gene_name": "DNA ligase 3",
  "term_id": "GO:0006273",
  "gene_symbol": "LIG3",
  "gene": "UniProtKB:P49916"
}